extrinsic apoptotic signaling pathway [GO:0097191] (biological process) Definition: The series of molecular signals in which a signal is conveyed from the cell surface to trigger the apoptotic death of a cell. The pathway starts with either a ligand binding to a cell surface receptor, or a ligand being withdrawn from a cell surface receptor (e.g. in the case of signaling by dependence receptors), and ends when the execution phase of apoptosis is triggered. References: PMID:17340152 Sources: GOC:mtg_apoptosis, GOC:yaf Also known as: extrinsic apoptotic pathway, extrinsic apoptotic signalling pathway, death receptor-mediated apoptosis, extrinsic apoptosis, extrinsic apoptotic signaling pathway in presence of ligand Note: Fas acts as a death receptor with a role in apoptosis, but can also act as a non-apoptotic signal transducer. Relationships: is a type of cell surface receptor signaling pathway [GO:0007166]; is a type of apoptotic signaling pathway [GO:0097190] Subtypes: extrinsic apoptotic signaling pathway via death domain receptors [GO:0008625], extrinsic apoptotic signaling pathway in absence of ligand [GO:0097192], GO:1902178, GO:1990117 Regulation: regulated by regulation of extrinsic apoptotic signaling pathway [GO:2001236]; negatively regulated by negative regulation of extrinsic apoptotic signaling pathway [GO:2001237]; positively regulated by positive regulation of extrinsic apoptotic signaling pathway [GO:2001238]